{
  "gene_symbol": "RNF19A",
  "gene": "UniProtKB:Q9NV58",
  "term_id": "GO:0005737",
  "term_label": "cytoplasm",
  "gene_name": "E3 ubiquitin-protein ligase RNF19A"
}